synapse organization [GO:0050808] (biological process) Definition: A process that is carried out at the cellular level which results in the assembly, arrangement of constituent parts, or disassembly of a synapse, the junction between a neuron and a target (neuron, muscle, or secretory cell). Relationships: is a type of cell junction organization [GO:0034330] Also known as: synapse organisation, synapse development, synapse morphogenesis, synapse organization and biogenesis Subtypes: synapse assembly [GO:0007416], neuromuscular junction development [GO:0007528], establishment of synaptic specificity at neuromuscular junction [GO:0007529], synapse maturation [GO:0060074], synapse pruning [GO:0098883], maintenance of synapse structure [GO:0099558], modification of synaptic structure [GO:0099563], GO:0150089 Sources: GOC:ai, GOC:pr Regulation: regulated by regulation of synapse organization [GO:0050807]; negatively regulated by negative regulation of synapse organization [GO:1905809]